{
  "gene_symbol": "AGBL2",
  "gene": "UniProtKB:Q5U5Z8",
  "term_id": "GO:0015630",
  "gene_name": "Cytosolic carboxypeptidase 2",
  "term_label": "microtubule cytoskeleton"
}